thymine/thymine mispair binding [GO:0035487] (molecular function) Definition: Binding to a double-stranded DNA region containing a T/T mispair. Also known as: T/T mispair binding Relationships: is a type of mismatched DNA binding [GO:0030983] Sources: GOC:bf, GOC:jh